BAD-BCL-2 complex [GO:0097138] (cellular component) References: PMID:14634621 Sources: GOC:so Relationships: is_a Bcl-2 family protein complex [GO:0097136] Definition: A heterodimeric protein complex consisting of BAD and BCL-2, members of the Bcl-2 family of anti- and proapoptotic regulators.